{
  "term_id": "GO:0050808",
  "gene_name": "Beta-synuclein",
  "term_label": "synapse organization",
  "gene": "UniProtKB:Q16143",
  "gene_symbol": "SNCB"
}